endodermal-mesodermal cell signaling [GO:0003133] (BP) Also known as: endodermal-mesodermal cell signalling Relationships: is a type of cell-cell signaling [GO:0007267] Sources: GOC:mtg_heart Subtypes: endodermal-mesodermal cell signaling involved in heart induction [GO:0003134] Definition: Any process that mediates the transfer of information from endodermal cells to mesodermal cells.